{
  "gene": "UniProtKB:Q86YC3",
  "term_label": "sequestering of TGFbeta in extracellular matrix",
  "gene_name": "Transforming growth factor beta activator LRRC33",
  "gene_symbol": "NRROS",
  "term_id": "GO:0035583"
}